borate efflux transmembrane transporter activity [GO:0080139] (molecular function) Relationships: is a type of GO:0015562; is part of GO:0035445 References: PMID:18603465 Also known as: boron efflux transmembrane transporter activity Definition: Enables the transfer of borate from the inside of the cell to the outside of the cell across a membrane.